{
  "term_label": "Unknown biological process",
  "gene_name": "Probable gluconokinase",
  "gene": "UniProtKB:Q5T6J7",
  "term_id": "UNKNOWN:0002",
  "gene_symbol": "IDNK"
}